lens morphogenesis in camera-type eye [GO:0002089] (biological process) Definition: The process in which the anatomical structures of the lens are generated and organized. The lens is a transparent structure in the eye through which light is focused onto the retina. An example of this process is found in Mus musculus. Relationships: is a type of GO:0009653; is part of GO:0002088; is part of GO:0048593 Also known as: lens morphogenesis, lens morphogenesis in camera-style eye Sources: GOC:dph, GOC:mtg_sensu